pyrimidine deoxyribonucleoside monophosphate metabolic process [GO:0009176] (biological process) Definition: The chemical reactions and pathways involving pyrimidine deoxynucleoside monophosphate, a compound consisting of a pyrimidine base linked to a deoxyribose sugar esterified with phosphate on the sugar. Relationships: is a type of pyrimidine nucleoside monophosphate metabolic process [GO:0009129] Also known as: pyrimidine deoxyribonucleoside monophosphate metabolism Subtypes: GO:0009177, pyrimidine deoxyribonucleoside monophosphate catabolic process [GO:0009178], GO:0046063, dTMP metabolic process [GO:0046073], dUMP metabolic process [GO:0046078] Sources: GOC:go_curators, ISBN:0198506732